{
  "term_id": "GO:0016020",
  "gene_symbol": "CMTM4",
  "gene": "UniProtKB:Q8IZR5",
  "gene_name": "CKLF-like MARVEL transmembrane domain-containing protein 4",
  "term_label": "membrane"
}